{
  "term_id": "UNKNOWN:0001",
  "term_label": "Unknown molecular function",
  "gene_symbol": "APOF",
  "gene_name": "Apolipoprotein F",
  "gene": "UniProtKB:Q13790"
}